{
  "term_label": "extracellular space",
  "gene_symbol": "LCN1P1",
  "gene": "UniProtKB:Q5VSP4",
  "term_id": "GO:0005615",
  "gene_name": "Putative lipocalin 1-like protein 1"
}